{
  "term_label": "plasma membrane",
  "gene": "UniProtKB:A6NDL8",
  "gene_symbol": "OR6C68",
  "gene_name": "Olfactory receptor 6C68",
  "term_id": "GO:0005886"
}